{
  "gene_name": "Leucine-rich repeat-containing protein 4C",
  "gene": "UniProtKB:Q9HCJ2",
  "term_label": "modulation of chemical synaptic transmission",
  "term_id": "GO:0050804",
  "gene_symbol": "LRRC4C"
}